CCL19-activated CCR7 signaling pathway [GO:0038119] (BP) Relationships: is a type of GO:0038115; is a type of C-C chemokine receptor CCR7 signaling pathway [GO:0038118] References: PMID:15059845 Sources: GOC:nhn, GOC:signaling Also known as: CCL19-activated CCR7 signalling pathway Definition: The series of molecular signals initiated by the binding of the C-C chemokine CCL19 to a C-C chemokine type 7 receptor (CCR7) on the surface of a target cell, and ending with the regulation of a downstream cellular process, e.g. transcription.